{
  "gene": "UniProtKB:Q8N339",
  "term_label": "detoxification of copper ion",
  "gene_symbol": "MT1M",
  "term_id": "GO:0010273",
  "gene_name": "Metallothionein-1M"
}